{
  "gene_name": "Putative ribosomal protein uL13-like",
  "gene_symbol": "RPL13AP3",
  "term_id": "UNKNOWN:0002",
  "gene": "UniProtKB:Q6NVV1",
  "term_label": "Unknown biological process"
}